{
  "term_label": "nucleus",
  "term_id": "GO:0005634",
  "gene_symbol": "ATF4",
  "gene_name": "Cyclic AMP-dependent transcription factor ATF-4",
  "gene": "UniProtKB:P18848"
}